{
  "term_id": "GO:0005739",
  "gene_name": "Protein NipSnap homolog 2",
  "gene_symbol": "NIPSNAP2",
  "gene": "UniProtKB:O75323",
  "term_label": "mitochondrion"
}